{
  "gene_symbol": "ARL6IP6",
  "term_id": "UNKNOWN:0003",
  "term_label": "Unknown cellular component",
  "gene_name": "ADP-ribosylation factor-like protein 6-interacting protein 6",
  "gene": "UniProtKB:Q8N6S5"
}